positive regulation of piRNA transcription [GO:0140543] (biological process) Definition: Any process that increases the frequency, rate or extent of the synthesis of piRNA. References: PMID:28847004 Relationships: is a type of positive regulation of DNA-templated transcription [GO:0045893]; is a type of regulation of piRNA transcription [GO:0140542]; positively regulates piRNA transcription [GO:0140541]